{
  "term_id": "GO:0005886",
  "gene_symbol": "OR6C6",
  "term_label": "plasma membrane",
  "gene": "UniProtKB:A6NF89",
  "gene_name": "Olfactory receptor 6C6"
}